{
  "gene": "UniProtKB:Q6W0C5",
  "gene_name": "Developmental pluripotency-associated protein 3",
  "term_label": "nucleus",
  "term_id": "GO:0005634",
  "gene_symbol": "DPPA3"
}